{
  "gene_symbol": "GDPD4",
  "gene_name": "Glycerophosphodiester phosphodiesterase domain-containing protein 4",
  "gene": "UniProtKB:Q6W3E5",
  "term_label": "membrane",
  "term_id": "GO:0016020"
}